{
  "term_label": "cell adhesion molecule binding",
  "gene_symbol": "EZR",
  "gene": "UniProtKB:P15311",
  "gene_name": "Ezrin",
  "term_id": "GO:0050839"
}